{
  "term_label": "endoplasmic reticulum",
  "gene": "UniProtKB:Q92685",
  "gene_name": "Dol-P-Man:Man(5)GlcNAc(2)-PP-Dol alpha-1,3-mannosyltransferase",
  "term_id": "GO:0005783",
  "gene_symbol": "ALG3"
}